{
  "gene_symbol": "SLC25A41",
  "gene": "UniProtKB:Q8N5S1",
  "term_label": "Unknown cellular component",
  "term_id": "UNKNOWN:0003",
  "gene_name": "Mitochondrial carrier protein SCaMC-3L"
}